{
  "gene_symbol": "WT1",
  "gene": "UniProtKB:P19544",
  "gene_name": "Wilms tumor protein",
  "term_id": "GO:0006357",
  "term_label": "regulation of transcription by RNA polymerase II"
}